{
  "term_id": "UNKNOWN:0002",
  "gene": "UniProtKB:Q5T6C5",
  "gene_symbol": "ATXN7L2",
  "gene_name": "Ataxin-7-like protein 2",
  "term_label": "Unknown biological process"
}